{
  "gene_name": "NT-3 growth factor receptor",
  "term_label": "neurotrophin receptor activity",
  "term_id": "GO:0005030",
  "gene_symbol": "NTRK3",
  "gene": "UniProtKB:Q16288"
}